{
  "term_id": "GO:0004197",
  "gene_name": "Cysteine protease ATG4D",
  "gene_symbol": "ATG4D",
  "term_label": "cysteine-type endopeptidase activity",
  "gene": "UniProtKB:Q86TL0"
}